Pup ligase activity [GO:0061664] (molecular function) Definition: Catalysis of the transfer of Pup to a substrate protein via the reaction X-Pup + S = X + S-Pup, where X is either an E2 or E3 enzyme, the X-Pup linkage is a thioester bond, and the S-Pup linkage is an isopeptide bond between the C-terminal amino acid of Pup and the epsilon-amino group of lysine residues in the substrate. Sources: GOC:dph Also known as: E3 Relationships: is a type of ubiquitin-like protein ligase activity [GO:0061659]; is a type of Pup transferase activity [GO:0072496]